{
  "gene_symbol": "SPDYE11",
  "gene": "UniProtKB:P0DTA3",
  "term_label": "protein kinase binding",
  "gene_name": "Putative speedy protein E11",
  "term_id": "GO:0019901"
}